symbiont-mediated suppression of host mRNA splicing [GO:0046780] (biological process) Also known as: suppression by virus of host splicing factor activity, negative regulation by virus of host mRNA splicing, suppression by virus of host mRNA splicing, viral dispersion of host splicing factors, viral inhibition of host mRNA splicing Definition: A process in which a symbiont inhibits or disrupts the splicing of host mRNA, thus interfering with normal host protein production. The host is defined as the larger of the organisms involved in a symbiotic interaction. References: PMID:12660167, PMID:19729513 Relationships: is a type of symbiont-mediated suppression of host mRNA processing [GO:0039524]